telomerase holoenzyme complex [GO:0005697] (cellular component) Definition: Telomerase is a ribonucleoprotein enzyme complex, with a minimal catalytic core composed of a catalytic reverse transcriptase subunit and an RNA subunit that provides the template for telomeric DNA addition. In vivo, the holoenzyme complex often contains additional subunits. References: PMID:11884619 Relationships: is a type of nuclear protein-containing complex [GO:0140513]; is_a catalytic complex [GO:1902494]; is a type of ribonucleoprotein complex [GO:1990904] Subtypes: telomerase catalytic core complex [GO:0000333]